{
  "term_id": "GO:0005886",
  "gene_name": "Olfactory receptor 2A1_2A42",
  "gene": "UniProtKB:Q8NGT9",
  "term_label": "plasma membrane",
  "gene_symbol": "OR2A1"
}